{
  "term_label": "Unknown biological process",
  "gene_name": "Cilia- and flagella-associated protein 97",
  "term_id": "UNKNOWN:0002",
  "gene": "UniProtKB:Q9P2B7",
  "gene_symbol": "CFAP97"
}